{
  "gene_symbol": "NTRK3",
  "gene": "UniProtKB:Q16288",
  "gene_name": "NT-3 growth factor receptor",
  "term_id": "GO:0030424",
  "term_label": "axon"
}